{
  "gene": "UniProtKB:P52789",
  "gene_name": "Hexokinase-2",
  "term_label": "glycolytic process",
  "term_id": "GO:0006096",
  "gene_symbol": "HK2"
}